{
  "gene_name": "Importin-4",
  "gene_symbol": "IPO4",
  "term_id": "GO:0005737",
  "term_label": "cytoplasm",
  "gene": "UniProtKB:Q8TEX9"
}